regulation of T cell receptor signaling pathway [GO:0050856] (biological process) Definition: Any process that modulates the frequency, rate or extent of signaling pathways initiated by the cross-linking of an antigen receptor on a T cell. Relationships: is a type of GO:0050854; regulates GO:0050852 Sources: GOC:ai Subtypes: GO:0050860, positive regulation of T cell receptor signaling pathway [GO:0050862] Also known as: regulation of T lymphocyte receptor signaling pathway, regulation of T lymphocyte receptor signalling pathway, regulation of T-cell receptor signaling pathway, regulation of T-cell receptor signalling pathway, regulation of T-lymphocyte receptor signaling pathway, regulation of T-lymphocyte receptor signalling pathway, regulation of TCR signaling pathway